salicin transport [GO:0042948] (BP) Sources: GOC:jl Relationships: is a type of beta-glucoside transport [GO:0015759]; is a type of GO:0015850 Definition: The directed movement of salicin (saligenin-beta-D-glucopyranoside), a glucoside of o-hydroxybenzylalcohol, into, out of or within a cell, or between cells, by means of some agent such as a transporter or pore.